{
  "gene_name": "Synaptotagmin-11",
  "gene_symbol": "SYT11",
  "gene": "UniProtKB:Q9BT88",
  "term_id": "GO:0099502",
  "term_label": "calcium-dependent activation of synaptic vesicle fusion"
}